{
  "gene_name": "Tyrosine-protein phosphatase non-receptor type 13",
  "gene": "UniProtKB:Q12923",
  "term_id": "GO:1904890",
  "gene_symbol": "PTPN13",
  "term_label": "negative regulation of excitatory synapse assembly"
}